negative regulation of glial cell-derived neurotrophic factor receptor signaling pathway involved in ureteric bud formation [GO:2000734] (biological process) Relationships: is a type of negative regulation of signal transduction [GO:0009968]; is a type of GO:2000733; negatively regulates GO:2000701 Also known as: negative regulation of GDNF receptor signaling pathway of ureteric bud formation, negative regulation of glial cell derived neurotrophic factor receptor signaling pathway of ureteric bud formation, negative regulation of glial cell line-derived neurotrophic factor receptor signalling pathway of ureteric bud formation, negative regulation of glial cell-derived neurotrophic factor receptor signaling pathway of ureteric bud formation, negative regulation of glial cell-derived neurotrophic factor receptor signalling pathway of ureteric bud formation Definition: Any process that stops, prevents or reduces the frequency, rate or extent of glial cell-derived neurotrophic factor receptor signaling pathway involved in ureteric bud formation. Sources: GOC:obol